{
  "gene_name": "Lysoplasmalogenase",
  "gene_symbol": "TMEM86B",
  "gene": "UniProtKB:Q8N661",
  "term_label": "D-lysine 5,6-aminomutase activity",
  "term_id": "GO:0047826"
}